{
  "term_id": "GO:0000423",
  "term_label": "mitophagy",
  "gene_symbol": "ULK3",
  "gene_name": "Serine_threonine-protein kinase ULK3",
  "gene": "UniProtKB:Q6PHR2"
}